{
  "gene_symbol": "DYNAP",
  "gene": "UniProtKB:Q8N1N2",
  "term_label": "Unknown molecular function",
  "gene_name": "Dynactin-associated protein",
  "term_id": "UNKNOWN:0001"
}